{
  "gene": "UniProtKB:P11168",
  "gene_symbol": "SLC2A2",
  "term_label": "plasma membrane",
  "gene_name": "Solute carrier family 2, facilitated glucose transporter member 2",
  "term_id": "GO:0005886"
}